{
  "gene": "UniProtKB:Q8N3I7",
  "term_id": "GO:0034464",
  "gene_symbol": "BBS5",
  "gene_name": "Bardet-Biedl syndrome 5 protein",
  "term_label": "BBSome"
}